DnaA-Dps complex [GO:1990084] (cellular component) Relationships: is a type of replication inhibiting complex [GO:1990078] Definition: A protein complex that negatively regulates strand-opening at the origin of replication, thereby interfering with replication initiation. This complex is thought to be involved in the regulation of replication under oxidative stress conditions. In E. coli, this complex is composed of DnaA and Dps. References: PMID:18284581 Sources: GOC:bhm